{
  "gene_name": "Glutamate receptor ionotropic, NMDA 2B",
  "term_label": "NMDA glutamate receptor activity",
  "gene_symbol": "GRIN2B",
  "term_id": "GO:0004972",
  "gene": "UniProtKB:Q13224"
}